{
  "term_id": "GO:0005737",
  "gene_symbol": "SASH3",
  "term_label": "cytoplasm",
  "gene_name": "SAM and SH3 domain-containing protein 3",
  "gene": "UniProtKB:O75995"
}